positive regulation of nervous system development [GO:0051962] (biological process) Subtypes: positive regulation of neurogenesis [GO:0050769], GO:0051965 Relationships: is a type of positive regulation of developmental process [GO:0051094]; is a type of positive regulation of multicellular organismal process [GO:0051240]; is a type of regulation of nervous system development [GO:0051960]; positively regulates nervous system development [GO:0007399] Sources: GOC:ai Definition: Any process that activates, maintains or increases the frequency, rate or extent of nervous system development, the origin and formation of nervous tissue. Also known as: up regulation of nervous system development, up-regulation of nervous system development, upregulation of nervous system development, activation of nervous system development, stimulation of nervous system development